{
  "gene": "UniProtKB:P11049",
  "term_id": "UNKNOWN:0002",
  "gene_symbol": "CD37",
  "term_label": "Unknown biological process",
  "gene_name": "Leukocyte antigen CD37"
}